{
  "term_label": "olfactory receptor activity",
  "gene_name": "Olfactory receptor 4S1",
  "term_id": "GO:0004984",
  "gene": "UniProtKB:Q8NGB4",
  "gene_symbol": "OR4S1"
}